{
  "gene_symbol": "TMEM129",
  "term_id": "UNKNOWN:0002",
  "term_label": "Unknown biological process",
  "gene_name": "E3 ubiquitin-protein ligase TM129",
  "gene": "UniProtKB:A0AVI4"
}